{
  "gene_name": "Zinc finger protein with KRAB and SCAN domains 8",
  "term_label": "RNA polymerase II cis-regulatory region sequence-specific DNA binding",
  "gene_symbol": "ZKSCAN8",
  "gene": "UniProtKB:Q15776",
  "term_id": "GO:0000978"
}